{
  "gene": "UniProtKB:Q13614",
  "term_id": "GO:0004438",
  "gene_symbol": "MTMR2",
  "term_label": "phosphatidylinositol-3-phosphate phosphatase activity",
  "gene_name": "Myotubularin-related protein 2"
}